{
  "term_id": "GO:0005737",
  "term_label": "cytoplasm",
  "gene": "UniProtKB:Q8NDL9",
  "gene_symbol": "AGBL5",
  "gene_name": "Cytosolic carboxypeptidase-like protein 5"
}